{
  "gene_symbol": "ADH4",
  "term_id": "GO:0051903",
  "gene_name": "All-trans-retinol dehydrogenase [NAD(+)] ADH4",
  "term_label": "S-(hydroxymethyl)glutathione dehydrogenase [NAD(P)+] activity",
  "gene": "UniProtKB:P08319"
}